{
  "gene": "UniProtKB:Q58HT5",
  "gene_symbol": "AWAT1",
  "term_id": "GO:0005789",
  "gene_name": "Acyl-CoA wax alcohol acyltransferase 1",
  "term_label": "endoplasmic reticulum membrane"
}